{
  "gene_symbol": "PRODH2",
  "term_label": "mitochondrion",
  "term_id": "GO:0005739",
  "gene": "UniProtKB:Q9UF12",
  "gene_name": "Hydroxyproline dehydrogenase"
}